alpha-glucan, water dikinase activity [GO:0050521] (molecular function) Also known as: a-glucan, water dikinase activity, ATP:alpha-glucan, water phosphotransferase activity, GWD, alpha-glucan,water dikinase activity, starch-related R1 protein activity Relationships: is a type of kinase activity [GO:0016301]; is a type of phosphotransferase activity, paired acceptors [GO:0016781] Sources: RHEA:11668 Definition: Catalysis of the reaction: [(1->4)-alpha-D-glucosyl](n) + n ATP + n H2O = [(1->4)-6-phospho-alpha-D-glucosyl](n) + n AMP + 2n H+ + n phosphate.